{
  "gene_name": "Teratocarcinoma-derived growth factor 1",
  "gene_symbol": "TDGF1",
  "term_label": "cell surface",
  "gene": "UniProtKB:P13385",
  "term_id": "GO:0009986"
}